embryo implantation [GO:0007566] (biological process) Relationships: is a type of GO:0022414; is part of GO:0007275; is part of female pregnancy [GO:0007565] References: PMID:10882512 Sources: GOC:isa_complete Also known as: blastocyst implantation Definition: Attachment of the blastocyst to the uterine lining.